{
  "gene": "UniProtKB:A6NJT0",
  "gene_name": "Homeobox protein unc-4 homolog",
  "gene_symbol": "UNCX",
  "term_id": "GO:0010468",
  "term_label": "regulation of gene expression"
}